{
  "gene_name": "Low affinity immunoglobulin gamma Fc region receptor III-B",
  "term_id": "GO:0001788",
  "term_label": "antibody-dependent cellular cytotoxicity",
  "gene_symbol": "FCGR3B",
  "gene": "UniProtKB:O75015"
}